{
  "gene_name": "Epithelial discoidin domain-containing receptor 1",
  "gene_symbol": "DDR1",
  "term_label": "plasma membrane",
  "term_id": "GO:0005886",
  "gene": "UniProtKB:Q08345"
}